{
  "term_id": "GO:0004984",
  "gene_name": "Olfactory receptor 4A5",
  "gene": "UniProtKB:Q8NH83",
  "term_label": "olfactory receptor activity",
  "gene_symbol": "OR4A5"
}